{
  "term_id": "UNKNOWN:0003",
  "term_label": "Unknown cellular component",
  "gene_name": "Putative uncharacterized protein FLJ31958",
  "gene": "UniProtKB:Q96MT0",
  "gene_symbol": "Q96MT0"
}